{
  "gene_name": "Small nuclear ribonucleoprotein E",
  "term_label": "precatalytic spliceosome",
  "gene": "UniProtKB:P62304",
  "term_id": "GO:0071011",
  "gene_symbol": "SNRPE"
}